{
  "gene_name": "Zinc finger and BTB domain-containing protein 42",
  "gene": "UniProtKB:B2RXF5",
  "gene_symbol": "ZBTB42",
  "term_id": "GO:0005634",
  "term_label": "nucleus"
}